trihydroxyferuloyl spermidine:S-adenosyl-L-methionine O-methyltransferase activity [GO:0080077] (molecular function) Definition: Catalysis of the transfer of a methyl group from S-adenosyl-L-methionine to the oxygen atom of a trihydroxyferuloyl spermidine molecule. References: PMID:19077165 Relationships: is a type of O-methyltransferase activity [GO:0008171]